{
  "gene": "UniProtKB:Q8TBZ2",
  "term_id": "GO:0006897",
  "term_label": "endocytosis",
  "gene_name": "MYCBP-associated protein",
  "gene_symbol": "MYCBPAP"
}